{
  "term_label": "ubiquitin protein ligase activity",
  "gene_symbol": "RFFL",
  "gene": "UniProtKB:Q8WZ73",
  "term_id": "GO:0061630",
  "gene_name": "E3 ubiquitin-protein ligase rififylin"
}